{
  "term_label": "positive regulation of transcription by RNA polymerase II",
  "gene": "UniProtKB:Q9ULH7",
  "gene_symbol": "MRTFB",
  "gene_name": "Myocardin-related transcription factor B",
  "term_id": "GO:0045944"
}